{
  "gene_name": "Adenylosuccinate synthetase isozyme 1",
  "gene_symbol": "ADSS1",
  "term_id": "GO:0004019",
  "term_label": "adenylosuccinate synthase activity",
  "gene": "UniProtKB:Q8N142"
}